insulin metabolic process [GO:1901142] (biological process) Definition: The chemical reactions and pathways involving insulin. Relationships: is a type of protein metabolic process [GO:0019538] Also known as: insulin metabolism Subtypes: insulin processing [GO:0030070], insulin catabolic process [GO:1901143] Sources: GOC:TermGenie